{
  "gene": "UniProtKB:A0A0B4J235",
  "gene_symbol": "TRAV13-2",
  "term_label": "Unknown cellular component",
  "term_id": "UNKNOWN:0003",
  "gene_name": "T cell receptor alpha variable 13-2"
}